{
  "gene_name": "Mediator of RNA polymerase II transcription subunit 25",
  "gene_symbol": "MED25",
  "term_id": "GO:0005667",
  "term_label": "transcription regulator complex",
  "gene": "UniProtKB:Q71SY5"
}